tetrahydrofolylpolyglutamate biosynthetic process [GO:0046901] (biological process) Also known as: folic acid-containing compound polyglutamylation, THF polyglutamylation, tetrahydrofolate polyglutamylation, tetrahydrofolyl-[Glu](n) biosynthesis, tetrahydrofolyl-[Glu](n) biosynthetic process, tetrahydrofolylpolyglutamate anabolism, tetrahydrofolylpolyglutamate biosynthesis, tetrahydrofolylpolyglutamate formation, tetrahydrofolylpolyglutamate synthesis Relationships: is a type of folic acid-containing compound biosynthetic process [GO:0009396]; is a type of tetrahydrofolylpolyglutamate metabolic process [GO:0046900] Definition: The chemical reactions and pathways resulting in the formation of tetrahydrofolylpolyglutamate, a folate derivative comprising tetrahydrofolate attached to a chain of glutamate residues. Sources: GOC:ai